{
  "gene": "UniProtKB:Q9NRH3",
  "gene_symbol": "TUBG2",
  "gene_name": "Tubulin gamma-2 chain",
  "term_label": "GTP binding",
  "term_id": "GO:0005525"
}